{
  "term_id": "UNKNOWN:0001",
  "term_label": "Unknown molecular function",
  "gene_symbol": "ALG13",
  "gene": "UniProtKB:Q9NP73",
  "gene_name": "Putative bifunctional UDP-N-acetylglucosamine transferase and deubiquitinase ALG13"
}